Kv4.1-DPP6 channel complex [GO:0071198] (cellular component) References: PMID:15911355 Also known as: Kv4.1-DPPX channel complex Relationships: is_a voltage-gated potassium channel complex [GO:0008076] Definition: A voltage-gated potassium channel complex that contains the peptidase-related protein DPP6 associated with the channel via interaction with the Kv alpha subunit 4.1.